anterior lateral line ganglion development [GO:0048907] (biological process) Definition: The process whose specific outcome is the progression of the anterior lateral line ganglion over time, from its formation to the mature structure. The anterior lateral line ganglion develops from cranial ectodermal placodes situated between the eye and ear. Also known as: gALL development Sources: ISBN:0125296509 Relationships: is a type of lateral line ganglion development [GO:0048890]; is part of anterior lateral line system development [GO:0048898]